{
  "gene": "UniProtKB:P23945",
  "term_label": "follicle-stimulating hormone receptor activity",
  "gene_name": "Follicle-stimulating hormone receptor",
  "term_id": "GO:0004963",
  "gene_symbol": "FSHR"
}